{
  "gene": "UniProtKB:Q53HL2",
  "gene_name": "Borealin",
  "term_label": "Unknown molecular function",
  "term_id": "UNKNOWN:0001",
  "gene_symbol": "CDCA8"
}